{
  "term_label": "negative regulation of circadian rhythm",
  "term_id": "GO:0042754",
  "gene_name": "Circadian clock protein PASD1",
  "gene": "UniProtKB:Q8IV76",
  "gene_symbol": "PASD1"
}